{
  "gene": "UniProtKB:A2RUB6",
  "term_label": "microtubule binding",
  "gene_symbol": "CCDC66",
  "gene_name": "Coiled-coil domain-containing protein 66",
  "term_id": "GO:0008017"
}